plant cell papilla [GO:0090395] (cellular component) Note: Part of papilla cell (PO:0025166), which is a shoot epidermal cell (PO:0025165) in plants. Replaces the obsolete term papillae (PO:0002001). Definition: A cell projection that is a short, rounded projection from a plant epidermal cell. Subtypes: GO:0090396, GO:0090397, trichome papilla [GO:0090705] Relationships: is a type of cell projection [GO:0042995] Sources: GOC:tb